{
  "gene_name": "Poly [ADP-ribose] polymerase tankyrase-1",
  "term_label": "nucleus",
  "gene_symbol": "TNKS",
  "term_id": "GO:0005634",
  "gene": "UniProtKB:O95271"
}